carcinine import across plasma membrane [GO:1905130] (BP) Relationships: is a type of GO:0015695; is a type of GO:0042886; is a type of azole transmembrane transport [GO:0045117]; is a type of GO:0072337; is_a GO:0098739 References: PMID:26653853, PMID:26713872 Sources: GOC:TermGenie, GOC:dph, GO_REF:0000075 Definition: The directed movement of carcinine from outside of a cell, across the plasma membrane and into the cytosol.